{
  "term_id": "GO:0004691",
  "gene_name": "cAMP-dependent protein kinase catalytic subunit beta",
  "gene": "UniProtKB:P22694",
  "gene_symbol": "PRKACB",
  "term_label": "cAMP-dependent protein kinase activity"
}